{
  "term_id": "GO:0005737",
  "term_label": "cytoplasm",
  "gene_symbol": "TSNAXIP1",
  "gene_name": "Translin-associated factor X-interacting protein 1",
  "gene": "UniProtKB:Q2TAA8"
}